ciliary neurotrophic factor receptor complex [GO:0070110] (cellular component) Relationships: is_a plasma membrane signaling receptor complex [GO:0098802] Definition: A protein complex that acts as a receptor for the cytokine ciliary neurotrophic factor (CNTF). In humans the receptor complex is a hexamer composed of two molecules each of CNTF and CNTFR and one molecule each of gp130 and LIFR. References: PMID:12707266 Sources: GOC:BHF, GOC:mah, GOC:rl